{
  "gene_name": "Serine_threonine-protein kinase N3",
  "term_id": "UNKNOWN:0003",
  "gene_symbol": "PKN3",
  "term_label": "Unknown cellular component",
  "gene": "UniProtKB:Q6P5Z2"
}